{
  "term_label": "plasma membrane",
  "gene": "UniProtKB:Q6UWI2",
  "term_id": "GO:0005886",
  "gene_symbol": "PARM1",
  "gene_name": "Prostate androgen-regulated mucin-like protein 1"
}